{
  "term_label": "mitochondrial L-ornithine transmembrane transport",
  "gene": "UniProtKB:Q9Y619",
  "gene_name": "Mitochondrial ornithine transporter 1",
  "gene_symbol": "SLC25A15",
  "term_id": "GO:1990575"
}